{
  "gene_name": "Uncharacterized protein FLJ43738",
  "gene_symbol": "Q6ZUG5",
  "gene": "UniProtKB:Q6ZUG5",
  "term_label": "Unknown molecular function",
  "term_id": "UNKNOWN:0001"
}